{
  "gene_name": "Protein transport protein Sec31A",
  "term_id": "GO:0007029",
  "term_label": "endoplasmic reticulum organization",
  "gene": "UniProtKB:O94979",
  "gene_symbol": "SEC31A"
}